{
  "gene": "UniProtKB:Q9BZF2",
  "gene_symbol": "OSBPL7",
  "gene_name": "Oxysterol-binding protein-related protein 7",
  "term_label": "cytosol",
  "term_id": "GO:0005829"
}